N-terminal peptidyl-proline methylation [GO:0035568] (biological process) Subtypes: N-terminal peptidyl-proline dimethylation [GO:0018016] Relationships: is a type of N-terminal protein amino acid methylation [GO:0006480]; is a type of peptidyl-proline modification [GO:0018208] Definition: The methylation of the N-terminal proline of proteins. References: PMID:20668449 Sources: RESID:AA0419